{
  "term_label": "protein sumoylation",
  "gene_name": "E3 SUMO-protein ligase PIAS3",
  "term_id": "GO:0016925",
  "gene": "UniProtKB:Q9Y6X2",
  "gene_symbol": "PIAS3"
}